{
  "gene": "UniProtKB:Q6Q0C0",
  "gene_name": "E3 ubiquitin-protein ligase TRAF7",
  "term_label": "regulation of ERK1 and ERK2 cascade",
  "term_id": "GO:0070372",
  "gene_symbol": "TRAF7"
}